nuclear receptor-mediated corticosteroid signaling pathway [GO:0031958] (biological process) Subtypes: nuclear receptor-mediated mineralocorticoid signaling pathway [GO:0031959], nuclear receptor-mediated glucocorticoid signaling pathway [GO:0042921] Definition: A nuclear receptor-mediated signaling pathway initiated by a corticosteroid binding to an intracellular receptor of the nuclear receptor protein family, and ending with regulation of a downstream cellular process, e.g. transcription. References: PMID:11027914, PMID:12606724 Also known as: corticosteroid receptor signalling pathway, intracellular corticosteroid receptor signaling pathway Relationships: is a type of GO:0030518